{
  "gene_symbol": "WRN",
  "gene_name": "Bifunctional 3'-5' exonuclease_ATP-dependent helicase WRN",
  "gene": "UniProtKB:Q14191",
  "term_id": "GO:0005634",
  "term_label": "nucleus"
}